imaginal disc-derived genitalia morphogenesis [GO:0048805] (biological process) Subtypes: imaginal disc-derived male genitalia morphogenesis [GO:0048803], GO:0048804 Also known as: genital morphogenesis Definition: The process in which the anatomical structures of genitalia are generated and organized from the genital imaginal disc. Sources: GOC:ai, GOC:sensu Relationships: is a type of post-embryonic genitalia morphogenesis [GO:0035126]; is part of genital disc morphogenesis [GO:0007483]; is part of imaginal disc-derived genitalia development [GO:0007484]